negative regulation of antigen processing and presentation of peptide or polysaccharide antigen via MHC class II [GO:0002581] (biological process) Subtypes: negative regulation of antigen processing and presentation of peptide antigen via MHC class II [GO:0002587], GO:0002602 Relationships: is a type of negative regulation of antigen processing and presentation [GO:0002578]; is_a regulation of antigen processing and presentation of peptide or polysaccharide antigen via MHC class II [GO:0002580]; negatively regulates antigen processing and presentation of peptide or polysaccharide antigen via MHC class II [GO:0002504] Also known as: down regulation of antigen processing and presentation of peptide or polysaccharide antigen via MHC class II, down-regulation of antigen processing and presentation of peptide or polysaccharide antigen via MHC class II, downregulation of antigen processing and presentation of peptide or polysaccharide antigen via MHC class II, negative regulation of peptide or polysaccharide antigen processing and presentation via MHC class II, inhibition of antigen processing and presentation of peptide or polysaccharide antigen via MHC class II Definition: Any process that stops, prevents, or reduces the frequency, rate, or extent of antigen processing and presentation of antigen (peptide or polysaccharide) via MHC class II. Sources: GOC:add